{
  "gene_symbol": "PLD6",
  "gene_name": "Mitochondrial cardiolipin hydrolase",
  "term_label": "mitochondrion",
  "term_id": "GO:0005739",
  "gene": "UniProtKB:Q8N2A8"
}